{
  "gene_name": "Uncharacterized protein CXorf51A",
  "gene_symbol": "CXorf51A",
  "term_id": "UNKNOWN:0003",
  "term_label": "Unknown cellular component",
  "gene": "UniProtKB:A0A1B0GTR3"
}